{
  "term_id": "GO:0000977",
  "gene_name": "Zinc finger protein 44",
  "term_label": "RNA polymerase II transcription regulatory region sequence-specific DNA binding",
  "gene_symbol": "ZNF44",
  "gene": "UniProtKB:P15621"
}